{
  "term_id": "GO:0042393",
  "gene": "UniProtKB:Q96GD3",
  "term_label": "histone binding",
  "gene_symbol": "SCMH1",
  "gene_name": "Polycomb protein SCMH1"
}